{
  "term_label": "adaptive immune response",
  "gene_symbol": "IFNG",
  "gene": "UniProtKB:P01579",
  "gene_name": "Interferon gamma",
  "term_id": "GO:0002250"
}